{
  "term_label": "catalytic step 2 spliceosome",
  "gene_symbol": "MAGOHB",
  "term_id": "GO:0071013",
  "gene_name": "Protein mago nashi homolog 2",
  "gene": "UniProtKB:Q96A72"
}